ABC-type amino acid transporter activity [GO:0015424] (molecular function) Relationships: is a type of amino acid transmembrane transporter activity [GO:0015171]; is a type of GO:0140359 Definition: Enables the transfer of a solute or solutes from one side of a membrane to the other according to the reaction: ATP + H2O + amino acid(out/in) = ADP + phosphate + amino acid(in/out). Also known as: ATP-dependent amino acid transmembrane transporter activity, amino acid-transporting ATPase activity, amino acid ABC transporter, ATPase-coupled amino acid transmembrane transporter activity, amino acid-exporting ATPase activity, amino acid-importing ATPase activity Subtypes: ATPase-coupled nonpolar-amino acid transporter activity [GO:0015425], ATPase-coupled polar amino acid-transporter activity [GO:0015426], ABC-type cysteine transporter activity [GO:0033230], ABC-type D-methionine transporter activity [GO:0033232] Sources: GOC:ai, GOC:mah